{
  "term_id": "GO:0036092",
  "term_label": "phosphatidylinositol-3-phosphate biosynthetic process",
  "gene_symbol": "PIK3CD",
  "gene_name": "Phosphatidylinositol 4,5-bisphosphate 3-kinase catalytic subunit delta isoform",
  "gene": "UniProtKB:O00329"
}